{
  "gene_name": "Heat shock protein HSP 90-alpha A2",
  "term_label": "protein folding",
  "gene": "UniProtKB:Q14568",
  "gene_symbol": "HSP90AA2P",
  "term_id": "GO:0006457"
}